trans-synaptic signaling by neuropeptide, modulating synaptic transmission [GO:0099551] (biological process) Subtypes: GO:0099083 Relationships: is a type of trans-synaptic signaling by neuropeptide [GO:0099540]; is a type of trans-synaptic signaling, modulating synaptic transmission [GO:0099550] Definition: Cell-cell signaling between presynapse and postsynapse, via the vesicular release and reception of neuropeptide molecules, that modulates the synaptic transmission properties of the synapse. Sources: GOC:dos Note: Note that this term was created for the SynGO project, and will be obsoleted when the SynGO annotations are made in Noctua.